{
  "gene_symbol": "HHLA3",
  "gene_name": "HERV-H LTR-associating protein 3",
  "term_id": "UNKNOWN:0001",
  "term_label": "Unknown molecular function",
  "gene": "UniProtKB:Q9XRX5"
}